{
  "gene": "UniProtKB:Q14507",
  "term_id": "UNKNOWN:0001",
  "gene_symbol": "EDDM3A",
  "gene_name": "Epididymal secretory protein E3-alpha",
  "term_label": "Unknown molecular function"
}